{
  "term_label": "Unknown cellular component",
  "gene_symbol": "STK32A",
  "gene": "UniProtKB:Q8WU08",
  "term_id": "UNKNOWN:0003",
  "gene_name": "Serine_threonine-protein kinase 32A"
}